{
  "gene_symbol": "CYP2A6",
  "term_label": "oxidoreductase activity, acting on paired donors, with incorporation or reduction of molecular oxygen, reduced flavin or flavoprotein as one donor, and incorporation of one atom of oxygen",
  "term_id": "GO:0016712",
  "gene": "UniProtKB:P11509",
  "gene_name": "Cytochrome P450 2A6"
}